{
  "term_label": "endoplasmic reticulum",
  "gene_symbol": "UGT1A6",
  "gene": "UniProtKB:P19224",
  "gene_name": "UDP-glucuronosyltransferase 1-6",
  "term_id": "GO:0005783"
}